{
  "term_label": "late endosome to vacuole transport",
  "gene_name": "Charged multivesicular body protein 2a",
  "term_id": "GO:0045324",
  "gene_symbol": "CHMP2A",
  "gene": "UniProtKB:O43633"
}